{
  "gene": "UniProtKB:Q96LX8",
  "gene_name": "Zinc finger protein 597",
  "gene_symbol": "ZNF597",
  "term_label": "nucleus",
  "term_id": "GO:0005634"
}